positive regulation of androst-4-ene-3,17-dione biosynthetic process [GO:1903456] (biological process) References: PMID:24399684 Sources: GOC:TermGenie, GOC:mr, GO_REF:0000058 Definition: Any process that activates or increases the frequency, rate or extent of androst-4-ene-3,17-dione biosynthetic process. Relationships: is a type of positive regulation of steroid biosynthetic process [GO:0010893]; is a type of positive regulation of small molecule metabolic process [GO:0062013]; is a type of regulation of androst-4-ene-3,17-dione biosynthetic process [GO:1903454]; positively regulates GO:1903449 Also known as: positive regulation of androst-4-ene-3,17-dione anabolism, positive regulation of androst-4-ene-3,17-dione biosynthesis, positive regulation of androst-4-ene-3,17-dione formation, positive regulation of androst-4-ene-3,17-dione synthesis, positive regulation of androstenedione biosynthetic process, up regulation of androst-4-ene-3,17-dione anabolism, up regulation of androst-4-ene-3,17-dione biosynthesis, up regulation of androst-4-ene-3,17-dione biosynthetic process, up regulation of androst-4-ene-3,17-dione formation, up regulation of androst-4-ene-3,17-dione synthesis, up regulation of androstenedione biosynthetic process, up-regulation of androst-4-ene-3,17-dione anabolism, up-regulation of androst-4-ene-3,17-dione biosynthesis, up-regulation of androst-4-ene-3,17-dione biosynthetic process, up-regulation of androst-4-ene-3,17-dione formation, up-regulation of androst-4-ene-3,17-dione synthesis, up-regulation of androstenedione biosynthetic process, upregulation of androst-4-ene-3,17-dione anabolism, upregulation of androst-4-ene-3,17-dione biosynthesis, upregulation of androst-4-ene-3,17-dione biosynthetic process, upregulation of androst-4-ene-3,17-dione formation, upregulation of androst-4-ene-3,17-dione synthesis, upregulation of androstenedione biosynthetic process, activation of androst-4-ene-3,17-dione anabolism, activation of androst-4-ene-3,17-dione biosynthesis, activation of androst-4-ene-3,17-dione biosynthetic process, activation of androst-4-ene-3,17-dione formation, activation of androst-4-ene-3,17-dione synthesis, activation of androstenedione